cyclic-nucleotide phosphodiesterase activity [GO:0004112] (molecular function) Definition: Catalysis of the reaction: a nucleoside cyclic phosphate + H2O = a nucleoside phosphate. Sources: GOC:mah Relationships: is a type of phosphoric diester hydrolase activity [GO:0008081] Subtypes: GO:0004113, 3',5'-cyclic-nucleotide phosphodiesterase activity [GO:0004114], GO:0008663 Regulation: negatively regulated by negative regulation of cyclic-nucleotide phosphodiesterase activity [GO:0051344]; RO_0002213 by cyclic nucleotide phosphodiesterase activator activity [GO:0170005]